{
  "term_id": "GO:0005886",
  "gene_symbol": "CALCR",
  "gene": "UniProtKB:P30988",
  "term_label": "plasma membrane",
  "gene_name": "Calcitonin receptor"
}